{
  "gene_symbol": "RPAP3",
  "gene_name": "RNA polymerase II-associated protein 3",
  "term_label": "Unknown cellular component",
  "term_id": "UNKNOWN:0003",
  "gene": "UniProtKB:Q9H6T3"
}